{
  "gene_name": "Zinc finger RNA-binding protein 2",
  "term_label": "Unknown cellular component",
  "gene": "UniProtKB:Q9UPR6",
  "term_id": "UNKNOWN:0003",
  "gene_symbol": "ZFR2"
}